{
  "term_label": "endomembrane system",
  "term_id": "GO:0012505",
  "gene": "UniProtKB:P14672",
  "gene_symbol": "SLC2A4",
  "gene_name": "Solute carrier family 2, facilitated glucose transporter member 4"
}